{
  "gene_symbol": "C12orf4",
  "term_label": "cytoplasm",
  "gene": "UniProtKB:Q9NQ89",
  "gene_name": "Protein C12orf4",
  "term_id": "GO:0005737"
}